{
  "term_id": "GO:0006357",
  "gene_symbol": "MSX2",
  "gene": "UniProtKB:P35548",
  "term_label": "regulation of transcription by RNA polymerase II",
  "gene_name": "Homeobox protein MSX-2"
}